{
  "gene": "UniProtKB:P05451",
  "term_label": "growth factor activity",
  "term_id": "GO:0008083",
  "gene_name": "Lithostathine-1-alpha",
  "gene_symbol": "REG1A"
}